succinylglutamate desuccinylase activity [GO:0009017] (molecular function) Sources: EC:3.5.1.96, RHEA:15169 Also known as: N2-succinylglutamate desuccinylase activity, AstE, N-succinyl-L-glutamate amidohydrolase activity, SGDS Definition: Catalysis of the reaction: N-succinyl-L-glutamate + H2O = L-glutamate + succinate. Relationships: is a type of hydrolase activity, acting on carbon-nitrogen (but not peptide) bonds, in linear amides [GO:0016811]